{
  "term_label": "cell surface",
  "gene_symbol": "KLRC3",
  "gene_name": "NKG2-E type II integral membrane protein",
  "term_id": "GO:0009986",
  "gene": "UniProtKB:Q07444"
}